cAMP catabolic process [GO:0006198] (biological process) Relationships: is a type of purine ribonucleotide catabolic process [GO:0009154]; is a type of cyclic nucleotide catabolic process [GO:0009214]; is a type of cAMP metabolic process [GO:0046058] Definition: The chemical reactions and pathways resulting in the breakdown of the nucleotide cAMP (cyclic AMP, adenosine 3',5'-cyclophosphate). Sources: ISBN:0198506732 Also known as: 3',5' cAMP catabolic process, 3',5' cAMP catabolism, 3',5'-cAMP catabolic process, 3',5'-cAMP catabolism, adenosine 3',5'-cyclophosphate catabolic process, adenosine 3',5'-cyclophosphate catabolism, cAMP breakdown, cAMP catabolism, cAMP degradation, cyclic AMP catabolic process, cyclic AMP catabolism